{
  "term_label": "Unknown molecular function",
  "gene": "UniProtKB:Q86YD7",
  "term_id": "UNKNOWN:0001",
  "gene_symbol": "FAM90A1",
  "gene_name": "Protein FAM90A1"
}